type 1 mitophagy [GO:0180045] (biological process) Relationships: is a type of mitophagy [GO:0000423] Definition: The selective autophagy process in which a functional mitochondrion is degraded by macroautophagy to provide metabolic precursors during nutrient deprivation or to remove mitochondria in excess of metabolic needs. References: PMID:25009776 Sources: GOC:vw